{
  "gene_symbol": "ZMYM3",
  "gene": "UniProtKB:Q14202",
  "term_id": "UNKNOWN:0001",
  "term_label": "Unknown molecular function",
  "gene_name": "Zinc finger MYM-type protein 3"
}